{
  "gene_symbol": "ANG",
  "term_label": "innate immune response",
  "gene_name": "Angiogenin",
  "gene": "UniProtKB:P03950",
  "term_id": "GO:0045087"
}